{
  "gene": "UniProtKB:Q5QGT7",
  "gene_name": "Receptor-transporting protein 2",
  "term_label": "protein insertion into membrane",
  "gene_symbol": "RTP2",
  "term_id": "GO:0051205"
}